{
  "term_id": "GO:0005771",
  "gene": "UniProtKB:P59074",
  "term_label": "multivesicular body",
  "gene_name": "Putative charged multivesicular body protein 4B-like protein CHMP4BP1",
  "gene_symbol": "CHMP4BP1"
}